centriole elongation [GO:0061511] (biological process) References: PMID:21576394 Sources: GOC:dph Regulation: regulated by GO:1903722; negatively regulated by negative regulation of centriole elongation [GO:1903723]; positively regulated by positive regulation of centriole elongation [GO:1903724] Relationships: is a type of cell cycle process [GO:0022402]; is part of centriole replication [GO:0007099] Definition: The centrosome organization process by which a centriole increases in length as part of the process of replication.